{
  "term_id": "GO:0032869",
  "term_label": "cellular response to insulin stimulus",
  "gene_name": "DENN domain-containing protein 4C",
  "gene": "UniProtKB:Q5VZ89",
  "gene_symbol": "DENND4C"
}